{
  "gene_symbol": "PLEKHA7",
  "gene_name": "Pleckstrin homology domain-containing family A member 7",
  "term_label": "cell-cell adhesion mediated by cadherin",
  "term_id": "GO:0044331",
  "gene": "UniProtKB:Q6IQ23"
}